{
  "gene_name": "V-type proton ATPase catalytic subunit A",
  "term_label": "proton transmembrane transport",
  "gene_symbol": "ATP6V1A",
  "term_id": "GO:1902600",
  "gene": "UniProtKB:P38606"
}